{
  "term_id": "GO:0051082",
  "gene_symbol": "HEATR3",
  "gene": "UniProtKB:Q7Z4Q2",
  "term_label": "unfolded protein binding",
  "gene_name": "HEAT repeat-containing protein 3"
}